lateral attachment of mitotic spindle microtubules to kinetochore [GO:0099607] (biological process) References: PMID:26258632, PMID:26705896 Relationships: is a type of attachment of mitotic spindle microtubules to kinetochore [GO:0051315] Regulation: regulated by regulation of lateral attachment of mitotic spindle microtubules to kinetochore [GO:1905115]; positively regulated by GO:1905116 Definition: The cellular process in which sister chromatids become laterally attached to spindle microtubules as part of mitotic metaphase plate congression. Attachment precedes migration along microtubules towards the spindle equator (metaphase plate).